ectoderm formation [GO:0001705] (biological process) Definition: The formation of ectoderm during gastrulation. Sources: GOC:go_curators Relationships: is a type of formation of primary germ layer [GO:0001704]; is part of ectoderm development [GO:0007398]